{
  "gene_name": "Protein SGT1 homolog",
  "gene_symbol": "SUGT1",
  "gene": "UniProtKB:Q9Y2Z0",
  "term_label": "Unknown biological process",
  "term_id": "UNKNOWN:0002"
}